{
  "gene": "UniProtKB:Q6QNY1",
  "gene_name": "Biogenesis of lysosome-related organelles complex 1 subunit 2",
  "term_label": "endosomal transport",
  "term_id": "GO:0016197",
  "gene_symbol": "BLOC1S2"
}